{
  "gene": "UniProtKB:Q9Y616",
  "gene_name": "Interleukin-1 receptor-associated kinase 3",
  "gene_symbol": "IRAK3",
  "term_label": "nucleus",
  "term_id": "GO:0005634"
}